regulation of C-C chemokine receptor CCR7 signaling pathway [GO:1903080] (BP) References: PMID:11602640 Sources: GOC:BHF, GOC:TermGenie, GOC:rl, GO_REF:0000058 Definition: Any process that modulates the frequency, rate or extent of C-C chemokine receptor CCR7 signaling pathway. Also known as: regulation of C-C chemokine receptor CCR7 signalling pathway, regulation of CCR7 signaling pathway Relationships: is a type of GO:0070099; regulates C-C chemokine receptor CCR7 signaling pathway [GO:0038118] Subtypes: negative regulation of C-C chemokine receptor CCR7 signaling pathway [GO:1903081], positive regulation of C-C chemokine receptor CCR7 signaling pathway [GO:1903082]